positive regulation of R8 cell spacing in compound eye [GO:0045748] (biological process) Also known as: positive regulation of R8 spacing, up regulation of R8 spacing, up-regulation of R8 spacing, upregulation of R8 spacing, activation of R8 spacing, stimulation of R8 spacing Definition: Any process that activates or enforces the correct R8 cell spacing in a compound eye. Relationships: is a type of regulation of R8 cell spacing in compound eye [GO:0045468] Sources: GOC:dph, GOC:go_curators, GOC:tb